{
  "term_id": "GO:0070129",
  "gene": "UniProtKB:Q9BT17",
  "term_label": "regulation of mitochondrial translation",
  "gene_name": "Mitochondrial ribosome-associated GTPase 1",
  "gene_symbol": "MTG1"
}